{
  "gene_symbol": "GTPBP3",
  "term_id": "GO:0002098",
  "gene_name": "tRNA modification GTPase GTPBP3, mitochondrial",
  "term_label": "tRNA wobble uridine modification",
  "gene": "UniProtKB:Q969Y2"
}